{
  "gene": "UniProtKB:Q9BT73",
  "gene_name": "Proteasome assembly chaperone 3",
  "gene_symbol": "PSMG3",
  "term_label": "Unknown molecular function",
  "term_id": "UNKNOWN:0001"
}